de-etiolation [GO:0009704] (biological process) Definition: The greening response of plants grown in the dark (etiolated) as a result of chloroplast biogenesis and the accumulation of chlorophyll. Relationships: is a type of response to light stimulus [GO:0009416]; is part of photomorphogenesis [GO:0009640] Sources: GOC:lr